{
  "gene_name": "Solute carrier family 40 member 1",
  "gene_symbol": "SLC40A1",
  "term_label": "iron ion transmembrane transport",
  "gene": "UniProtKB:Q9NP59",
  "term_id": "GO:0034755"
}